hormone receptor binding [GO:0051427] (molecular function) Subtypes: growth hormone receptor binding [GO:0005131], GO:0051428 Sources: GOC:ai Definition: Binding to a receptor for a hormone. Relationships: is a type of signaling receptor binding [GO:0005102]